{
  "gene": "UniProtKB:P0C7W0",
  "gene_name": "Proline-rich protein 29",
  "term_label": "Unknown molecular function",
  "gene_symbol": "PRR29",
  "term_id": "UNKNOWN:0001"
}